dGMP kinase activity [GO:0050316] (molecular function) Also known as: T2-induced deoxynucleotide kinase activity, ATP:(d)NMP phosphotransferase activity Relationships: is a type of GO:0047507 Definition: Catalysis of the reaction: dGMP + ATP = dGDP + ADP. Sources: RHEA:12697